{
  "gene_symbol": "XRCC2",
  "term_id": "GO:0005657",
  "term_label": "replication fork",
  "gene_name": "DNA repair protein XRCC2",
  "gene": "UniProtKB:O43543"
}